{
  "gene_symbol": "NLRP5",
  "term_id": "GO:0005634",
  "term_label": "nucleus",
  "gene_name": "NACHT, LRR and PYD domains-containing protein 5",
  "gene": "UniProtKB:P59047"
}